{
  "term_label": "nucleus",
  "gene_symbol": "HOXB8",
  "term_id": "GO:0005634",
  "gene": "UniProtKB:P17481",
  "gene_name": "Homeobox protein Hox-B8"
}